endoplasmic reticulum cisternal network assembly [GO:0071784] (biological process) References: PMID:16469703, PMID:20434336 Sources: GOC:mah Definition: The aggregation, arrangement and bonding together of a set of components to form the endoplasmic reticulum (ER) cisternal network. The ER cisternal network is the ER part that comprises the membranes with low curvature in cross-section. Also known as: ER cisternal network assembly, ER cisternal network formation, endoplasmic reticulum cisternal network formation Relationships: is a type of cellular component assembly [GO:0022607]; is a type of endoplasmic reticulum cisternal network organization [GO:0071783]